negative regulation of long-day photoperiodism, flowering [GO:0048579] (biological process) Also known as: down regulation of long-day photoperiodism, flowering, down-regulation of long-day photoperiodism, flowering, downregulation of long-day photoperiodism, flowering, inhibition of long-day photoperiodism, flowering Relationships: is a type of GO:0048581; is a type of negative regulation of response to stimulus [GO:0048585]; is_a regulation of long-day photoperiodism, flowering [GO:0048586]; RO_0002212 long-day photoperiodism, flowering [GO:0048574] Sources: GOC:jid, GOC:pj, ISBN:0582015952, ISBN:0697037754, ISBN:0709408862 Definition: Any process that stops, prevents or reduces long-day photoperiodism, where the response associated with the photoperiodism is flowering. Flowering is defined by the switch from the vegetative to the reproductive phase.